{
  "term_id": "GO:0005737",
  "gene_symbol": "UBA1",
  "gene_name": "Ubiquitin-like modifier-activating enzyme 1",
  "gene": "UniProtKB:P22314",
  "term_label": "cytoplasm"
}